{
  "term_label": "antigen processing and presentation of endogenous peptide antigen via MHC class Ib",
  "term_id": "GO:0002476",
  "gene_symbol": "HLA-B",
  "gene": "UniProtKB:P01889",
  "gene_name": "HLA class I histocompatibility antigen, B alpha chain"
}